{
  "term_label": "regulation of transcription by RNA polymerase II",
  "gene": "UniProtKB:P12980",
  "term_id": "GO:0006357",
  "gene_symbol": "LYL1",
  "gene_name": "Protein lyl-1"
}